inner cell mass cell proliferation [GO:0001833] (biological process) Note: See also the Anatomical Dictionary for Mouse Development ontology terms 'TS4, inner cell mass ; EMAP:14' and 'TS5, inner cell mass ; EMAP:24'. Sources: GOC:dph, GOC:isa_complete, ISBN:0124020607, ISBN:0198542771 Definition: The proliferation of cells in the inner cell mass. Relationships: is a type of cell population proliferation [GO:0008283]; is part of blastocyst growth [GO:0001832]